{
  "gene_name": "Histone-arginine methyltransferase METTL23",
  "gene_symbol": "METTL23",
  "gene": "UniProtKB:Q86XA0",
  "term_label": "cytoplasm",
  "term_id": "GO:0005737"
}